vesicle tethering to endoplasmic reticulum [GO:0099044] (biological process) Definition: The initial, indirect interaction between a transport vesicle membrane and the membrane of the endoplasmic reticulum. This interaction is mediated by tethering factors (or complexes), which interact with both membranes. Interaction can occur via direct binding to membrane phospholipids or membrane proteins, or via binding to vesicle coat proteins. This process is distinct from and prior fusion. Relationships: is a type of GO:0099022 References: PMID:27243008